{
  "term_label": "DNA-binding transcription factor activity, RNA polymerase II-specific",
  "gene_name": "Proto-oncogene c-Rel",
  "term_id": "GO:0000981",
  "gene": "UniProtKB:Q04864",
  "gene_symbol": "REL"
}